{
  "gene": "UniProtKB:O75223",
  "term_label": "gamma-glutamylcyclotransferase activity",
  "term_id": "GO:0003839",
  "gene_name": "Gamma-glutamylcyclotransferase",
  "gene_symbol": "GGCT"
}